inner ear receptor cell fate commitment [GO:0060120] (biological process) Subtypes: auditory receptor cell fate commitment [GO:0009912], vestibular receptor cell fate commitment [GO:0060115] Definition: The process in which a cell becomes committed to become an inner ear receptor cell. Also known as: inner ear hair cell fate commitment Sources: GOC:dph Relationships: is a type of neuron fate commitment [GO:0048663]; is part of inner ear receptor cell differentiation [GO:0060113]